{
  "gene_symbol": "NTRK2",
  "gene": "UniProtKB:Q16620",
  "term_label": "dendritic spine",
  "gene_name": "BDNF_NT-3 growth factors receptor",
  "term_id": "GO:0043197"
}